negative regulation of single-species biofilm formation in or on host organism [GO:1900229] (biological process) Definition: Any process that stops, prevents or reduces the frequency, rate or extent of single-species biofilm formation in or on host organism. Also known as: down regulation of single-species biofilm formation in or on host organism, down-regulation of single-species biofilm formation in or on host organism, downregulation of single-species biofilm formation in or on host organism, inhibition of single-species biofilm formation in or on host organism Sources: GOC:TermGenie, GOC:di Relationships: is a type of GO:1900191; is a type of regulation of single-species biofilm formation in or on host organism [GO:1900228]; negatively regulates GO:0044407